{
  "gene_name": "Zinc finger protein 69 homolog B",
  "term_id": "GO:0005634",
  "term_label": "nucleus",
  "gene": "UniProtKB:Q9UJL9",
  "gene_symbol": "ZFP69B"
}